{
  "gene": "UniProtKB:Q92564",
  "term_id": "GO:0000151",
  "gene_symbol": "DCUN1D4",
  "term_label": "ubiquitin ligase complex",
  "gene_name": "DCN1-like protein 4"
}